{
  "gene_symbol": "TRAJ28",
  "gene_name": "T cell receptor alpha joining 28 (Fragment)",
  "term_label": "Unknown cellular component",
  "term_id": "UNKNOWN:0003",
  "gene": "UniProtKB:A0A075B6X4"
}